{
  "term_id": "GO:0001707",
  "term_label": "mesoderm formation",
  "gene": "UniProtKB:Q0VG99",
  "gene_name": "Mesoderm posterior protein 2",
  "gene_symbol": "MESP2"
}